{
  "gene_symbol": "PAK1",
  "gene": "UniProtKB:Q13153",
  "gene_name": "Serine_threonine-protein kinase PAK 1",
  "term_label": "cell migration",
  "term_id": "GO:0016477"
}